{
  "term_id": "GO:0030127",
  "term_label": "COPII vesicle coat",
  "gene": "UniProtKB:O95487",
  "gene_name": "Protein transport protein Sec24B",
  "gene_symbol": "SEC24B"
}